{
  "term_id": "UNKNOWN:0003",
  "term_label": "Unknown cellular component",
  "gene_name": "Galectin-10",
  "gene": "UniProtKB:Q05315",
  "gene_symbol": "CLC"
}